{
  "gene": "UniProtKB:P0C7T7",
  "term_id": "UNKNOWN:0001",
  "term_label": "Unknown molecular function",
  "gene_symbol": "FRMD6-AS1",
  "gene_name": "Putative uncharacterized protein FRMD6-AS1"
}